{
  "term_label": "Unknown biological process",
  "gene_symbol": "DSN1",
  "gene_name": "Kinetochore-associated protein DSN1 homolog",
  "gene": "UniProtKB:Q9H410",
  "term_id": "UNKNOWN:0002"
}